nuclear mRNA surveillance of mRNP export [GO:0071032] (biological process) Definition: The set of processes involved in identifying and degrading incorrectly formed or aberrant nuclear mRNPs docked at the nuclear pore complex prior to export to the cytoplasm. References: PMID:18644474 Sources: GOC:dgf, GOC:krc Also known as: nuclear mRNA catabolic process of mRNAs in aberrant mRNPs, nuclear mRNA quality control of mRNAs in aberrant mRNPs Relationships: is a type of GO:0071028